{
  "gene_name": "NK1 transcription factor-related protein 1",
  "gene": "UniProtKB:Q15270",
  "term_label": "nucleus",
  "term_id": "GO:0005634",
  "gene_symbol": "NKX1-1"
}